{
  "gene_symbol": "RRH",
  "term_label": "plasma membrane",
  "term_id": "GO:0005886",
  "gene": "UniProtKB:O14718",
  "gene_name": "Visual pigment-like receptor peropsin"
}